{
  "term_label": "immune response",
  "gene_symbol": "SLAMF8",
  "gene": "UniProtKB:Q9P0V8",
  "gene_name": "SLAM family member 8",
  "term_id": "GO:0006955"
}